{
  "term_label": "axonogenesis",
  "gene_symbol": "SLITRK4",
  "gene": "UniProtKB:Q8IW52",
  "gene_name": "SLIT and NTRK-like protein 4",
  "term_id": "GO:0007409"
}